positive regulation of monocyte chemotactic protein-1 production [GO:0071639] (biological process) Also known as: positive regulation of CCL2 production, positive regulation of MCP-1 production Definition: Any process that activates or increases the frequency, rate, or extent of production of monocyte chemotactic protein-1. Sources: GOC:mah Relationships: is a type of GO:0032722; is a type of GO:0071637; positively regulates monocyte chemotactic protein-1 production [GO:0071605]